membrane macromolecule biosynthetic process [GO:0071710] (biological process) Sources: GOC:mah Definition: The chemical reactions and pathways resulting in the formation of a macromolecule destined to form part of a membrane in a cell. Relationships: is a type of macromolecule biosynthetic process [GO:0009059]; is part of membrane biogenesis [GO:0044091] Also known as: membrane macromolecule anabolism, membrane macromolecule biosynthesis, membrane macromolecule formation, membrane macromolecule synthesis